{
  "term_label": "spliceosomal complex",
  "gene_name": "Nucleolin",
  "gene": "UniProtKB:P19338",
  "gene_symbol": "NCL",
  "term_id": "GO:0005681"
}